negative regulation of nigerotriose transport [GO:1900358] (biological process) Definition: Any process that stops, prevents or reduces the frequency, rate or extent of nigerotriose transport. Sources: GOC:TermGenie, GOC:mengo_curators Also known as: down regulation of nigerotriose transport, down-regulation of nigerotriose transport, downregulation of nigerotriose transport, inhibition of nigerotriose transport Relationships: is a type of GO:0051051; is a type of regulation of nigerotriose transport [GO:1900357]; negatively regulates GO:2001091